{
  "gene_name": "Bcl-2-like protein 1",
  "term_id": "GO:0015267",
  "gene_symbol": "BCL2L1",
  "term_label": "channel activity",
  "gene": "UniProtKB:Q07817"
}